tRNA 4-thiouridine biosynthesis [GO:0002937] (biological process) Note: In E. coli, two genes are involved, nuvA (aka Thi) and NuvC (aka iscS) . NuvA converts the trNA into an unidentified intermediate in an ATP dependent manner. NucC catalyzes the second step, transferring the sulfur from cysteine to an unidentified intermediate. NuvC also participates in thiamine synthesis. Definition: The processes whereby a uridine residue in a tRNA is converted to 4-thiouridine. Typically 4-thiouridine is found at position 8, in many transfer RNAs. Sources: ISBN:155581073X Relationships: is a type of tRNA thio-modification [GO:0034227]